{
  "gene_name": "Cytosolic acyl coenzyme A thioester hydrolase",
  "term_id": "GO:0009062",
  "gene_symbol": "ACOT7",
  "gene": "UniProtKB:O00154",
  "term_label": "fatty acid catabolic process"
}